{
  "gene_symbol": "MIA3",
  "gene_name": "Transport and Golgi organization protein 1 homolog",
  "term_id": "UNKNOWN:0001",
  "gene": "UniProtKB:Q5JRA6",
  "term_label": "Unknown molecular function"
}